{
  "gene_symbol": "MDFIC",
  "gene": "UniProtKB:Q9P1T7",
  "gene_name": "MyoD family inhibitor domain-containing protein",
  "term_label": "cytoplasm",
  "term_id": "GO:0005737"
}